{
  "term_id": "GO:0000977",
  "gene_symbol": "STOX1",
  "gene": "UniProtKB:Q6ZVD7",
  "gene_name": "Storkhead-box protein 1",
  "term_label": "RNA polymerase II transcription regulatory region sequence-specific DNA binding"
}